{
  "gene_name": "Macrophage metalloelastase",
  "gene_symbol": "MMP12",
  "term_id": "UNKNOWN:0003",
  "term_label": "Unknown cellular component",
  "gene": "UniProtKB:P39900"
}